{
  "gene": "UniProtKB:O15392",
  "term_label": "Unknown molecular function",
  "gene_symbol": "BIRC5",
  "term_id": "UNKNOWN:0001",
  "gene_name": "Baculoviral IAP repeat-containing protein 5"
}